{
  "term_id": "UNKNOWN:0001",
  "gene_symbol": "LIMS3",
  "term_label": "Unknown molecular function",
  "gene": "UniProtKB:P0CW19",
  "gene_name": "LIM and senescent cell antigen-like-containing domain protein 3"
}